{
  "gene_symbol": "CHRNG",
  "term_id": "GO:0007268",
  "term_label": "chemical synaptic transmission",
  "gene": "UniProtKB:P07510",
  "gene_name": "Acetylcholine receptor subunit gamma"
}